protein localization to phagophore assembly site [GO:0034497] (biological process) Relationships: is a type of GO:0008104; is part of autophagosome assembly [GO:0000045] Sources: GOC:rb Definition: Any process in which a protein is transported to, or maintained at, the phagophore assembly site (PAS). Also known as: protein localisation to phagophore assembly site, protein localization to PAS, protein localization to pre-autophagosomal structure